{
  "term_id": "GO:0045218",
  "gene": "UniProtKB:Q6IQ23",
  "gene_symbol": "PLEKHA7",
  "term_label": "zonula adherens maintenance",
  "gene_name": "Pleckstrin homology domain-containing family A member 7"
}